{
  "term_id": "GO:0005737",
  "gene": "UniProtKB:Q96B67",
  "gene_symbol": "ARRDC3",
  "gene_name": "Arrestin domain-containing protein 3",
  "term_label": "cytoplasm"
}